{
  "gene_name": "Interleukin-10 receptor subunit beta",
  "gene_symbol": "IL10RB",
  "gene": "UniProtKB:Q08334",
  "term_label": "plasma membrane",
  "term_id": "GO:0005886"
}